{
  "gene_symbol": "FAM111A",
  "gene": "UniProtKB:Q96PZ2",
  "term_label": "protein-DNA covalent cross-linking repair",
  "term_id": "GO:0106300",
  "gene_name": "Serine protease FAM111A"
}